{
  "term_id": "UNKNOWN:0001",
  "term_label": "Unknown molecular function",
  "gene": "UniProtKB:Q9NRG9",
  "gene_name": "Aladin",
  "gene_symbol": "AAAS"
}